{
  "term_id": "UNKNOWN:0002",
  "term_label": "Unknown biological process",
  "gene_name": "WD repeat-containing protein 27",
  "gene_symbol": "WDR27",
  "gene": "UniProtKB:A2RRH5"
}